{
  "gene_name": "Beta-crystallin A2",
  "gene_symbol": "CRYBA2",
  "term_id": "GO:0005212",
  "gene": "UniProtKB:P53672",
  "term_label": "structural constituent of eye lens"
}